{
  "gene": "UniProtKB:P18846",
  "term_label": "DNA-binding transcription factor activity, RNA polymerase II-specific",
  "term_id": "GO:0000981",
  "gene_symbol": "ATF1",
  "gene_name": "Cyclic AMP-dependent transcription factor ATF-1"
}